methylglyoxal catabolic process [GO:0051596] (biological process) Relationships: is a type of methylglyoxal metabolic process [GO:0009438]; is a type of ketone catabolic process [GO:0042182]; is a type of aldehyde catabolic process [GO:0046185]; is a type of cellular detoxification of methylglyoxal [GO:0140041] Subtypes: methylglyoxal catabolic process to lactate [GO:0061727] Definition: The chemical reactions and pathways resulting in the breakdown of methylglyoxal, CH3-CO-CHO, the aldehyde of pyruvic acid. Sources: GOC:ai Also known as: methylglyoxal breakdown, methylglyoxal catabolism, methylglyoxal degradation